{
  "term_id": "GO:0031507",
  "term_label": "heterochromatin formation",
  "gene": "UniProtKB:Q99878",
  "gene_symbol": "H2AC14",
  "gene_name": "Histone H2A type 1-J"
}